{
  "gene_symbol": "OR8B2",
  "term_id": "GO:0005549",
  "term_label": "odorant binding",
  "gene_name": "Olfactory receptor 8B2",
  "gene": "UniProtKB:Q96RD0"
}